{
  "gene_symbol": "MAP3K2",
  "gene_name": "Mitogen-activated protein kinase kinase kinase 2",
  "term_id": "GO:0004674",
  "gene": "UniProtKB:Q9Y2U5",
  "term_label": "protein serine/threonine kinase activity"
}